{
  "gene": "UniProtKB:P84550",
  "term_id": "GO:0000981",
  "gene_symbol": "SKOR1",
  "gene_name": "SKI family transcriptional corepressor 1",
  "term_label": "DNA-binding transcription factor activity, RNA polymerase II-specific"
}